{
  "gene_symbol": "TRIM74",
  "gene_name": "Tripartite motif-containing protein 74",
  "term_id": "GO:0061630",
  "term_label": "ubiquitin protein ligase activity",
  "gene": "UniProtKB:Q86UV6"
}